{
  "gene_symbol": "HABP2",
  "term_label": "serine-type endopeptidase activity",
  "gene": "UniProtKB:Q14520",
  "term_id": "GO:0004252",
  "gene_name": "Hyaluronan-binding protein 2"
}